{
  "gene_name": "HLA class I histocompatibility antigen, alpha chain E",
  "gene": "UniProtKB:P13747",
  "term_label": "antigen processing and presentation of endogenous peptide antigen via MHC class I via ER pathway, TAP-independent",
  "term_id": "GO:0002486",
  "gene_symbol": "HLA-E"
}